AUU codon-amino acid adaptor activity [GO:0033433] (MF) Relationships: is a type of triplet codon-amino acid adaptor activity [GO:0030533] Note: Note that in the standard genetic code, ATT codes for isoleucine. Sources: GOC:mah Also known as: ATT codon-amino acid adaptor activity, isoleucine tRNA Definition: A triplet codon-amino acid adaptor activity that recognizes an AUU codon.